positive regulation of oxidative phosphorylation [GO:1903862] (biological process) References: PMID:10225962 Sources: GOC:TermGenie, GO_REF:0000058 Also known as: positive regulation of respiratory-chain phosphorylation, up regulation of oxidative phosphorylation, up regulation of respiratory-chain phosphorylation, up-regulation of oxidative phosphorylation, up-regulation of respiratory-chain phosphorylation, upregulation of oxidative phosphorylation, upregulation of respiratory-chain phosphorylation, activation of oxidative phosphorylation, activation of respiratory-chain phosphorylation Definition: Any process that activates or increases the frequency, rate or extent of oxidative phosphorylation. Relationships: is_a GO:0002082; is a type of positive regulation of cellular respiration [GO:1901857]; positively regulates GO:0006119